{
  "term_id": "GO:0007342",
  "gene_name": "Sperm equatorial segment protein 1",
  "gene": "UniProtKB:Q6UW49",
  "gene_symbol": "SPESP1",
  "term_label": "fusion of sperm to egg plasma membrane involved in single fertilization"
}